{
  "term_label": "transcription coactivator activity",
  "gene_symbol": "NCOA2",
  "gene": "UniProtKB:Q15596",
  "gene_name": "Nuclear receptor coactivator 2",
  "term_id": "GO:0003713"
}